{
  "term_id": "GO:0005737",
  "gene_symbol": "ANXA10",
  "term_label": "cytoplasm",
  "gene_name": "Annexin A10",
  "gene": "UniProtKB:Q9UJ72"
}